{
  "term_label": "mitochondrial intermembrane space",
  "gene_symbol": "COA4",
  "gene_name": "Cytochrome c oxidase assembly factor 4 homolog, mitochondrial",
  "term_id": "GO:0005758",
  "gene": "UniProtKB:Q9NYJ1"
}